{
  "term_id": "GO:0005615",
  "term_label": "extracellular space",
  "gene": "UniProtKB:Q92626",
  "gene_symbol": "PXDN",
  "gene_name": "Peroxidasin homolog"
}